{
  "term_label": "chondroitin-glucuronate 5-epimerase activity",
  "term_id": "GO:0047757",
  "gene": "UniProtKB:Q8IZU8",
  "gene_name": "Dermatan-sulfate epimerase-like protein",
  "gene_symbol": "DSEL"
}